{
  "gene_name": "Insulin gene enhancer protein ISL-2",
  "gene": "UniProtKB:Q96A47",
  "gene_symbol": "ISL2",
  "term_id": "GO:0000987",
  "term_label": "cis-regulatory region sequence-specific DNA binding"
}